{
  "gene": "UniProtKB:Q86X29",
  "gene_symbol": "LSR",
  "term_label": "establishment of blood-brain barrier",
  "gene_name": "Lipolysis-stimulated lipoprotein receptor",
  "term_id": "GO:0060856"
}